actin binding [GO:0003779] (molecular function) Definition: Binding to monomeric or multimeric forms of actin, including actin filaments. Sources: GOC:clt Also known as: membrane associated actin binding Relationships: is a type of cytoskeletal protein binding [GO:0008092] Subtypes: GO:0003785, actin filament binding [GO:0051015]